{
  "gene_name": "Immunoglobulin kappa variable 2D-29",
  "term_label": "immunoglobulin complex",
  "gene_symbol": "IGKV2D-29",
  "gene": "UniProtKB:A0A075B6S2",
  "term_id": "GO:0019814"
}